{
  "gene_name": "Lysosomal alpha-mannosidase",
  "gene": "UniProtKB:O00754",
  "gene_symbol": "MAN2B1",
  "term_label": "lysosome",
  "term_id": "GO:0005764"
}